{
  "gene_name": "RecQ-like DNA helicase BLM",
  "term_label": "cytoplasm",
  "term_id": "GO:0005737",
  "gene_symbol": "BLM",
  "gene": "UniProtKB:P54132"
}